{
  "gene_symbol": "ZNF311",
  "term_label": "RNA polymerase II cis-regulatory region sequence-specific DNA binding",
  "gene_name": "Zinc finger protein 311",
  "term_id": "GO:0000978",
  "gene": "UniProtKB:Q5JNZ3"
}